negative regulation of oxidative stress-induced neuron intrinsic apoptotic signaling pathway [GO:1903377] (biological process) Subtypes: negative regulation of hydrogen peroxide-induced neuron intrinsic apoptotic signaling pathway [GO:1903384] Also known as: down regulation of neuron intrinsic apoptotic signaling pathway in response to oxidative stress, down-regulation of neuron intrinsic apoptotic signaling pathway in response to oxidative stress, downregulation of neuron intrinsic apoptotic signaling pathway in response to oxidative stress, negative regulation of neuron intrinsic apoptotic signaling pathway in response to oxidative stress, negative regulation of oxidative stress-induced neuron apoptosis, inhibition of neuron intrinsic apoptotic signaling pathway in response to oxidative stress, down regulation of neuron apoptosis in response to oxidative stress, down-regulation of neuron apoptosis in response to oxidative stress, downregulation of neuron apoptosis in response to oxidative stress, inhibition of neuron apoptosis in response to oxidative stress, negative regulation of neuron apoptosis in response to oxidative stress, neuroprotection against oxidative stress-induced apoptosis, protection against oxidative stress-induced neuron apoptosis, protection against oxidative stress-induced neuronal apoptosis Definition: Any process that stops, prevents or reduces the frequency, rate or extent of oxidative stress-induced neuron intrinsic apoptotic signaling pathway. Relationships: is a type of negative regulation of neuron apoptotic process [GO:0043524]; is a type of negative regulation of oxidative stress-induced intrinsic apoptotic signaling pathway [GO:1902176]; is a type of GO:1903376; negatively regulates neuron intrinsic apoptotic signaling pathway in response to oxidative stress [GO:0036480] References: PMID:15790595 Sources: GOC:PARL, GOC:TermGenie, GOC:bf, GO_REF:0000058